{
  "gene": "UniProtKB:O00292",
  "term_id": "GO:0009948",
  "term_label": "anterior/posterior axis specification",
  "gene_name": "Left-right determination factor 2",
  "gene_symbol": "LEFTY2"
}